{
  "term_label": "Unknown cellular component",
  "gene": "UniProtKB:Q8WUF5",
  "term_id": "UNKNOWN:0003",
  "gene_symbol": "PPP1R13L",
  "gene_name": "RelA-associated inhibitor"
}